{
  "gene_name": "Zinc finger and BTB domain-containing protein 20",
  "term_label": "regulation of immune system process",
  "gene": "UniProtKB:Q9HC78",
  "term_id": "GO:0002682",
  "gene_symbol": "ZBTB20"
}